protein localization to nuclear pore [GO:0090204] (biological process) Also known as: protein localisation to nuclear pore Sources: GOC:dph, GOC:rb, GOC:tb Definition: A process in which a protein is transported to, or maintained in, a nuclear pore. Relationships: is_a protein localization to nuclear envelope [GO:0090435]